{
  "gene_name": "Transmembrane emp24 domain-containing protein 4",
  "term_label": "intracellular protein transport",
  "gene": "UniProtKB:Q7Z7H5",
  "gene_symbol": "TMED4",
  "term_id": "GO:0006886"
}